{
  "term_id": "GO:0005143",
  "gene_symbol": "IL12A",
  "gene": "UniProtKB:P29459",
  "term_label": "interleukin-12 receptor binding",
  "gene_name": "Interleukin-12 subunit alpha"
}